{
  "gene_name": "Lysosomal enzyme trafficking factor",
  "gene_symbol": "LYSET",
  "term_label": "Unknown molecular function",
  "gene": "UniProtKB:Q8N6I4",
  "term_id": "UNKNOWN:0001"
}